{
  "term_label": "protein transmembrane transporter activity",
  "gene_symbol": "TIMM17B",
  "gene_name": "Mitochondrial import inner membrane translocase subunit Tim17-B",
  "gene": "UniProtKB:O60830",
  "term_id": "GO:0008320"
}